{
  "term_id": "UNKNOWN:0001",
  "gene": "UniProtKB:P0DTF9",
  "gene_name": "PTTG1IP family member 2",
  "term_label": "Unknown molecular function",
  "gene_symbol": "PTTG1IP2"
}